{
  "term_label": "negative regulation of transcription by RNA polymerase II",
  "gene_name": "Melanoma-associated antigen E2",
  "gene": "UniProtKB:Q8TD90",
  "term_id": "GO:0000122",
  "gene_symbol": "MAGEE2"
}